{
  "term_id": "GO:0005739",
  "gene": "UniProtKB:Q53H12",
  "term_label": "mitochondrion",
  "gene_name": "Acylglycerol kinase, mitochondrial",
  "gene_symbol": "AGK"
}